{
  "gene_name": "Actin-like protein 8",
  "gene_symbol": "ACTL8",
  "term_label": "structural constituent of postsynaptic actin cytoskeleton",
  "gene": "UniProtKB:Q9H568",
  "term_id": "GO:0098973"
}